{
  "gene_name": "Transcription factor SOX-5",
  "gene_symbol": "SOX5",
  "term_id": "GO:0000978",
  "gene": "UniProtKB:P35711",
  "term_label": "RNA polymerase II cis-regulatory region sequence-specific DNA binding"
}